{
  "gene_symbol": "PCOLCE",
  "gene_name": "Procollagen C-endopeptidase enhancer 1",
  "term_id": "GO:0006508",
  "term_label": "proteolysis",
  "gene": "UniProtKB:Q15113"
}